{
  "term_label": "cytoplasm",
  "gene_symbol": "PARVG",
  "gene": "UniProtKB:Q9HBI0",
  "term_id": "GO:0005737",
  "gene_name": "Gamma-parvin"
}